negative regulation of pole plasm oskar mRNA localization [GO:0045855] (biological process) Definition: Any process that stops, prevents, or reduces the frequency, rate or extent of a process in which oskar mRNA is transported to, or maintained in, the oocyte pole plasm. Sources: GOC:go_curators Also known as: down regulation of pole plasm oskar mRNA localization, down-regulation of pole plasm oskar mRNA localization, downregulation of pole plasm oskar mRNA localization, negative regulation of oocyte pole plasm oskar mRNA localization, negative regulation of pole plasm oskar mRNA localisation, inhibition of pole plasm oskar mRNA localization Relationships: is a type of GO:0007317; is a type of GO:1904581; negatively regulates pole plasm oskar mRNA localization [GO:0045451]